{
  "gene_name": "Renin receptor",
  "gene": "UniProtKB:O75787",
  "term_id": "UNKNOWN:0001",
  "gene_symbol": "ATP6AP2",
  "term_label": "Unknown molecular function"
}